{
  "gene_symbol": "SLC4A8",
  "gene": "UniProtKB:Q2Y0W8",
  "term_id": "GO:0005886",
  "term_label": "plasma membrane",
  "gene_name": "Electroneutral sodium bicarbonate exchanger 1"
}